{
  "term_id": "GO:0003723",
  "gene": "UniProtKB:Q9BUL9",
  "gene_name": "Ribonuclease P protein subunit p25",
  "gene_symbol": "RPP25",
  "term_label": "RNA binding"
}